{
  "gene_symbol": "LRRC72",
  "term_id": "UNKNOWN:0002",
  "gene_name": "Leucine-rich repeat-containing protein 72",
  "gene": "UniProtKB:A6NJI9",
  "term_label": "Unknown biological process"
}